positive regulation of antifungal peptide secretion [GO:0002802] (biological process) Definition: Any process that activates or increases the frequency, rate, or extent of antifungal peptide secretion. Relationships: is a type of positive regulation of antimicrobial peptide secretion [GO:0002796]; is a type of regulation of antifungal peptide secretion [GO:0002800]; is a type of positive regulation of antifungal peptide production [GO:0002804]; RO_0002213 GO:0002782 Also known as: up regulation of antifungal peptide secretion, up-regulation of antifungal peptide secretion, upregulation of antifungal peptide secretion, activation of antifungal peptide secretion, stimulation of antifungal peptide secretion Sources: GOC:add